specific granule lumen [GO:0035580] (cellular component) References: PMID:7334549 Sources: GOC:bf Definition: The volume enclosed by the membrane of a specific granule, a granule with a membranous, tubular internal structure, found primarily in mature neutrophil cells. Most are released into the extracellular fluid. Specific granules contain lactoferrin, lysozyme, vitamin B12 binding protein and elastase. Relationships: is a type of secretory granule lumen [GO:0034774]; is part of GO:0042581 Also known as: secondary granule lumen